peptidyl-tyrosine modification [GO:0018212] (biological process) Subtypes: peptidyl-tyrosine sulfation [GO:0006478], GO:0018108, GO:0018251 Definition: The modification of peptidyl-tyrosine. Relationships: is a type of peptidyl-amino acid modification [GO:0018193] Sources: GOC:go_curators